paraxial mesodermal cell differentiation [GO:0048342] (biological process) Definition: The process in which a relatively unspecialized cell acquires the specialized features of a paraxial mesoderm cell. Sources: GOC:dgh Relationships: is_a mesodermal cell differentiation [GO:0048333]; is part of paraxial mesoderm formation [GO:0048341]